{
  "gene_symbol": "H2BC12L",
  "term_label": "nucleus",
  "term_id": "GO:0005634",
  "gene": "UniProtKB:P57053",
  "gene_name": "Histone H2B type F-S"
}